{
  "gene": "UniProtKB:Q9Y2H9",
  "gene_name": "Microtubule-associated serine_threonine-protein kinase 1",
  "gene_symbol": "MAST1",
  "term_id": "GO:0004674",
  "term_label": "protein serine/threonine kinase activity"
}